{
  "gene_name": "Protein BTG2",
  "gene": "UniProtKB:P78543",
  "term_id": "UNKNOWN:0001",
  "term_label": "Unknown molecular function",
  "gene_symbol": "BTG2"
}